{
  "gene_symbol": "TWF2",
  "gene_name": "Twinfilin-2",
  "term_id": "GO:0005884",
  "gene": "UniProtKB:Q6IBS0",
  "term_label": "actin filament"
}